{
  "gene_symbol": "ZNF583",
  "term_id": "GO:0005634",
  "gene_name": "Zinc finger protein 583",
  "term_label": "nucleus",
  "gene": "UniProtKB:Q96ND8"
}